protocatechuate catabolic process, meta-cleavage [GO:0019617] (biological process) Sources: MetaCyc:P184-PWY Also known as: protocatechuate breakdown, meta-cleavage, protocatechuate catabolic process to oxaloacetate and pyruvate, protocatechuate degradation, meta-cleavage, 3,4-dihydroxybenzoate catabolic process, meta-cleavage Relationships: is a type of pyruvate metabolic process [GO:0006090]; is a type of oxaloacetate metabolic process [GO:0006107]; is a type of 3,4-dihydroxybenzoate catabolic process [GO:0019619] Definition: The chemical reactions and pathways resulting in the breakdown of protocatechuate, the anion of 3,4-dihydroxybenzoic acid, to yield oxaloacetate and pyruvate.